{
  "gene": "UniProtKB:Q9UM07",
  "gene_symbol": "PADI4",
  "term_id": "GO:0005737",
  "term_label": "cytoplasm",
  "gene_name": "Protein-arginine deiminase type-4"
}